serotonin secretion, neurotransmission [GO:0060096] (biological process) Definition: The regulated release of serotonin by a cell, in which released serotonin acts as a neurotransmitter. Sources: GOC:dph Also known as: serotonin release, neurotransmission Relationships: is a type of GO:0001820; is_a neurotransmitter secretion [GO:0007269]